histone mRNA stem-loop binding complex [GO:0062073] (cellular component) References: PMID:18025107, PMID:23286197 Sources: GOC:bhm Also known as: SLBP-MIF4GD complex, SLBP-SLIP1 complex Relationships: is a type of GO:0032991; is part of GO:0005737 Definition: A protein-containing complex composed of a stem-loop binding protein (in most species SLBP) and its interacting partner (SLIP1 or MIF4GD in most species) that binds to the histone mRNA (hmRNA) 3-prime-stem-loop structure. Facilitates hmRNA translation initiation and may also be involved in its processing and nuclear export.